{
  "gene": "UniProtKB:Q9NQT6",
  "gene_name": "Fascin-3",
  "term_id": "GO:0051015",
  "gene_symbol": "FSCN3",
  "term_label": "actin filament binding"
}